{
  "gene": "UniProtKB:Q9NZJ4",
  "term_id": "GO:0030544",
  "term_label": "Hsp70 protein binding",
  "gene_name": "Sacsin",
  "gene_symbol": "SACS"
}